{
  "gene_symbol": "CDSN",
  "term_id": "GO:0098609",
  "term_label": "cell-cell adhesion",
  "gene": "UniProtKB:Q15517",
  "gene_name": "Corneodesmosin"
}